histone H3K79 methyltransferase activity [GO:0031151] (molecular function) Relationships: is a type of protein-lysine N-methyltransferase activity [GO:0016279]; is a type of histone H3 methyltransferase activity [GO:0140938] Subtypes: histone H3K79 monomethyltransferase activity [GO:0120505], histone H3K79 dimethyltransferase activity [GO:0120506], GO:0140956 References: PMID:15371351 Note: Comment: Note that the residue position corresponds to the canonical human H3 histone (UniProtKB:P84243); this residue is conserved across all eukaryotes. Residue 1 is the first residue following removal of the initiating Methionine (Met). Note that each histone is encoded by multiple genes, and sequences may vary across different genes within an organism. Also known as: histone H3K79 methylase activity, histone lysine N-methyltransferase activity (H3-K79 specific), histone methylase activity (H3-K79 specific), histone methyltransferase activity (H3-K79 specific), histone-H3K79 methyltransferase activity Definition: Catalysis of the reaction: S-adenosyl-L-methionine + histone H3 L-lysine (position 79) = S-adenosyl-L-homocysteine + histone H3 N6-methyl-L-lysine (position 79). This reaction is the addition of a methyl group to the lysine residue at position 79 of the histone H3 protein.